{
  "gene_symbol": "PDE4A",
  "gene_name": "cAMP-specific 3',5'-cyclic phosphodiesterase 4A",
  "gene": "UniProtKB:P27815",
  "term_id": "GO:0047555",
  "term_label": "3',5'-cyclic-GMP phosphodiesterase activity"
}